{
  "term_id": "UNKNOWN:0001",
  "gene": "UniProtKB:P01721",
  "gene_name": "Immunoglobulin lambda variable 6-57",
  "term_label": "Unknown molecular function",
  "gene_symbol": "IGLV6-57"
}